{
  "term_label": "SNAP receptor activity",
  "term_id": "GO:0005484",
  "gene": "UniProtKB:Q12981",
  "gene_symbol": "BNIP1",
  "gene_name": "Vesicle transport protein SEC20"
}